regulation of actin cytoskeleton organization [GO:0032956] (biological process) Definition: Any process that modulates the frequency, rate or extent of the formation, arrangement of constituent parts, or disassembly of cytoskeletal structures comprising actin filaments and their associated proteins. Also known as: regulation of actin cytoskeleton organisation, regulation of actin cytoskeleton organization and biogenesis Sources: GOC:mah Relationships: is a type of regulation of actin filament-based process [GO:0032970]; is a type of regulation of cytoskeleton organization [GO:0051493]; regulates actin cytoskeleton organization [GO:0030036] Subtypes: regulation of actin filament length [GO:0030832], regulation of myosin II filament organization [GO:0043519], GO:0090138, regulation of actomyosin structure organization [GO:0110020], regulation of actin filament organization [GO:0110053], GO:0120133